{
  "term_label": "U1 snRNA binding",
  "term_id": "GO:0030619",
  "gene": "UniProtKB:Q6P2Q9",
  "gene_name": "Pre-mRNA-processing-splicing factor 8",
  "gene_symbol": "PRPF8"
}